{
  "gene_name": "Transient receptor potential cation channel subfamily A member 1",
  "term_id": "GO:0005886",
  "term_label": "plasma membrane",
  "gene": "UniProtKB:O75762",
  "gene_symbol": "TRPA1"
}